{
  "gene_symbol": "ARNT2",
  "gene": "UniProtKB:Q9HBZ2",
  "term_label": "aryl hydrocarbon receptor complex",
  "term_id": "GO:0034751",
  "gene_name": "Aryl hydrocarbon receptor nuclear translocator 2"
}